{
  "gene_symbol": "PSMD10",
  "term_id": "GO:0061629",
  "term_label": "RNA polymerase II-specific DNA-binding transcription factor binding",
  "gene_name": "26S proteasome non-ATPase regulatory subunit 10",
  "gene": "UniProtKB:O75832"
}